{
  "gene_name": "Olfactory receptor 56A5",
  "term_label": "plasma membrane",
  "gene_symbol": "OR56A5",
  "term_id": "GO:0005886",
  "gene": "UniProtKB:P0C7T3"
}